cellular component organization or biogenesis [GO:0071840] (biological process) Subtypes: cellular component organization [GO:0016043], cellular component biogenesis [GO:0044085] Sources: GOC:mah Also known as: cellular component organisation or biogenesis, cellular component organisation or biogenesis at cellular level, cellular component organization or biogenesis at cellular level Note: Note that this term is in the subset of terms that should not be used for direct gene product annotation. Instead, select a child term or, if no appropriate child term exists, please request a new term. Direct annotations to this term may be amended during annotation QC. Relationships: is a type of GO:0009987 Definition: A process that results in the biosynthesis of constituent macromolecules, assembly, arrangement of constituent parts, or disassembly of a cellular component.